regulation of vasculature development [GO:1901342] (biological process) Sources: GOC:TermGenie Relationships: is_a regulation of multicellular organismal development [GO:2000026]; regulates GO:0001944 Subtypes: regulation of angioblast cell migration involved in selective angioblast sprouting [GO:0035477], GO:0045765, GO:0110079, negative regulation of vasculature development [GO:1901343], GO:1904018 Definition: Any process that modulates the frequency, rate or extent of vasculature development. Also known as: regulation of vascular system development